{
  "gene_symbol": "FGF8",
  "gene": "UniProtKB:P55075",
  "term_label": "type 1 fibroblast growth factor receptor binding",
  "gene_name": "Fibroblast growth factor 8",
  "term_id": "GO:0005105"
}